fast-twitch skeletal muscle fiber contraction [GO:0031443] (biological process) Regulation: regulated by regulation of fast-twitch skeletal muscle fiber contraction [GO:0031446]; RO_0002212 by negative regulation of fast-twitch skeletal muscle fiber contraction [GO:0031447]; RO_0002213 by positive regulation of fast-twitch skeletal muscle fiber contraction [GO:0031448] Also known as: fast-twitch skeletal fiber contraction, fast-twitch skeletal fibre contraction, fast-twitch skeletal muscle fibre contraction, fast-twitch skeletal myofiber contraction, fast-twitch skeletal myofibre contraction Definition: A process in which force is generated within fast-twitch skeletal muscle tissue, resulting in a change in muscle geometry. Force generation involves a chemo-mechanical energy conversion step that is carried out by the actin/myosin complex activity, which generates force through ATP hydrolysis. The fast-twitch skeletal muscle is characterized by fast time parameters, high force development and fatiguability. Relationships: is a type of twitch skeletal muscle contraction [GO:0014721] Sources: GOC:ef, GOC:mah, GOC:mtg_muscle